regulation of synaptic vesicle endocytosis [GO:1900242] (BP) Relationships: is a type of regulation of endocytosis [GO:0030100]; is a type of regulation of synaptic vesicle recycling [GO:1903421]; regulates synaptic vesicle endocytosis [GO:0048488] Subtypes: GO:1900243, positive regulation of synaptic vesicle endocytosis [GO:1900244] Also known as: regulation of synaptic vesicle retrieval Definition: Any process that modulates the frequency, rate or extent of synaptic vesicle endocytosis. Sources: GOC:BHF, GOC:TermGenie